{
  "term_label": "L-tyrosine catabolic process",
  "term_id": "GO:0006572",
  "gene_name": "4-hydroxyphenylpyruvate dioxygenase",
  "gene": "UniProtKB:P32754",
  "gene_symbol": "HPD"
}